{
  "gene_symbol": "FAHD2B",
  "term_id": "UNKNOWN:0002",
  "term_label": "Unknown biological process",
  "gene": "UniProtKB:Q6P2I3",
  "gene_name": "Fumarylacetoacetate hydrolase domain-containing protein 2B"
}